regulation of B cell anergy [GO:0002670] (biological process) Definition: Any process that modulates the frequency, rate, or extent of B cell anergy. Relationships: is a type of GO:0002661; is a type of regulation of lymphocyte anergy [GO:0002911]; regulates B cell anergy [GO:0002515] Subtypes: negative regulation of B cell anergy [GO:0002671], positive regulation of B cell anergy [GO:0002672], regulation of central B cell anergy [GO:0002914], regulation of peripheral B cell anergy [GO:0002917] Sources: GOC:add Also known as: regulation of B lymphocyte anergy, regulation of B-cell anergy, regulation of B-lymphocyte anergy